CAC codon-amino acid adaptor activity [GO:0033426] (molecular function) Also known as: histidine tRNA Definition: A triplet codon-amino acid adaptor activity that recognizes a CAC codon. Relationships: is a type of triplet codon-amino acid adaptor activity [GO:0030533] Sources: GOC:mah Note: Note that in the standard genetic code, CAC codes for histidine.